{
  "term_label": "cytoskeletal anchor activity",
  "gene_symbol": "BICD1",
  "gene_name": "Protein bicaudal D homolog 1",
  "gene": "UniProtKB:Q96G01",
  "term_id": "GO:0008093"
}